{
  "gene_symbol": "DGKK",
  "term_id": "GO:0005886",
  "gene_name": "Diacylglycerol kinase kappa",
  "gene": "UniProtKB:Q5KSL6",
  "term_label": "plasma membrane"
}